{
  "gene_name": "Olfactory receptor 1A2",
  "gene_symbol": "OR1A2",
  "term_id": "GO:0007165",
  "term_label": "signal transduction",
  "gene": "UniProtKB:Q9Y585"
}